{
  "gene_symbol": "APOD",
  "term_label": "lipid metabolic process",
  "gene_name": "Apolipoprotein D",
  "term_id": "GO:0006629",
  "gene": "UniProtKB:P05090"
}